{
  "term_id": "GO:0005634",
  "gene_name": "Transcription factor 19",
  "term_label": "nucleus",
  "gene": "UniProtKB:Q9Y242",
  "gene_symbol": "TCF19"
}